{
  "gene_name": "ADP-ribosylation factor-like protein 5A",
  "gene": "UniProtKB:Q9Y689",
  "term_id": "GO:0005737",
  "gene_symbol": "ARL5A",
  "term_label": "cytoplasm"
}